{
  "term_id": "GO:0006915",
  "gene_symbol": "PRUNE2",
  "term_label": "apoptotic process",
  "gene": "UniProtKB:Q8WUY3",
  "gene_name": "Protein prune homolog 2"
}